host cell synaptic vesicle [GO:0098584] (cellular component) Definition: A secretory organelle of a host cell, some 50 nm in diameter, of presynaptic nerve terminals; accumulates in high concentrations of neurotransmitters and secretes these into the synaptic cleft by fusion with the 'active zone' of the presynaptic plasma membrane. Relationships: is a type of host cell cytoplasmic vesicle [GO:0044161]; BFO_0000050 GO:0044221 Sources: GOC:dos